{
  "gene_symbol": "DRAP1",
  "term_id": "GO:0017054",
  "gene_name": "Dr1-associated corepressor",
  "gene": "UniProtKB:Q14919",
  "term_label": "negative cofactor 2 complex"
}